{
  "gene_symbol": "MAJIN",
  "gene_name": "Membrane-anchored junction protein",
  "term_id": "GO:0005637",
  "gene": "UniProtKB:Q3KP22",
  "term_label": "nuclear inner membrane"
}